{
  "term_label": "RNA binding",
  "gene": "UniProtKB:Q6P158",
  "gene_name": "Putative ATP-dependent RNA helicase DHX57",
  "term_id": "GO:0003723",
  "gene_symbol": "DHX57"
}